{
  "gene": "UniProtKB:Q8N9N2",
  "gene_name": "Activating signal cointegrator 1 complex subunit 1",
  "gene_symbol": "ASCC1",
  "term_id": "GO:0005634",
  "term_label": "nucleus"
}